{
  "term_id": "GO:0032922",
  "gene_name": "Class E basic helix-loop-helix protein 41",
  "gene_symbol": "BHLHE41",
  "gene": "UniProtKB:Q9C0J9",
  "term_label": "circadian regulation of gene expression"
}